{
  "gene_name": "Ubiquitin-like protein 4B",
  "gene_symbol": "UBL4B",
  "gene": "UniProtKB:Q8N7F7",
  "term_label": "Unknown molecular function",
  "term_id": "UNKNOWN:0001"
}